{
  "gene_symbol": "SLC25A40",
  "term_label": "Unknown molecular function",
  "gene": "UniProtKB:Q8TBP6",
  "gene_name": "Probable mitochondrial glutathione transporter SLC25A40",
  "term_id": "UNKNOWN:0001"
}